{
  "gene": "UniProtKB:P05129",
  "gene_symbol": "PRKCG",
  "term_id": "GO:0035556",
  "term_label": "intracellular signal transduction",
  "gene_name": "Protein kinase C gamma type"
}